{
  "gene": "UniProtKB:Q04671",
  "gene_name": "P protein",
  "gene_symbol": "OCA2",
  "term_id": "GO:0030318",
  "term_label": "melanocyte differentiation"
}